collagen type XXIII trimer [GO:1990322] (cellular component) References: PMID:17876790 Relationships: is a type of transmembrane collagen trimer [GO:0030936] Definition: A collagen homotrimer of alpha1(XXIII) chains; type XXIII collagen triple helices span the plasma membrane.